{
  "gene_name": "Testis-expressed protein 264",
  "term_id": "GO:0000421",
  "term_label": "autophagosome membrane",
  "gene": "UniProtKB:Q9Y6I9",
  "gene_symbol": "TEX264"
}